oxaloacetate(2-) transmembrane transport [GO:1902356] (biological process) Definition: The directed movement of oxaloacetate(2-) across a membrane. References: PMID:18682385 Sources: GOC:TermGenie, GOC:dph Relationships: is a type of oxaloacetate transport [GO:0015729]; is a type of carboxylic acid transmembrane transport [GO:1905039] Subtypes: GO:1990555